{
  "term_id": "GO:0022008",
  "gene_name": "Fibroblast growth factor 2",
  "gene": "UniProtKB:P09038",
  "term_label": "neurogenesis",
  "gene_symbol": "FGF2"
}